{
  "term_label": "RNA binding",
  "term_id": "GO:0003723",
  "gene_name": "rRNA_tRNA 2'-O-methyltransferase fibrillarin-like protein 1",
  "gene": "UniProtKB:A6NHQ2",
  "gene_symbol": "FBLL1"
}